positive regulation of smooth muscle hypertrophy [GO:1905149] (biological process) Definition: Any process that activates or increases the frequency, rate or extent of smooth muscle hypertrophy. Also known as: up regulation of smooth muscle hypertrophy, up-regulation of smooth muscle hypertrophy, upregulation of smooth muscle hypertrophy, activation of smooth muscle hypertrophy Relationships: is a type of positive regulation of muscle hypertrophy [GO:0014742]; is a type of GO:0014744; is a type of regulation of smooth muscle hypertrophy [GO:1905147]; positively regulates smooth muscle hypertrophy [GO:0014895] References: PMID:22161164 Sources: GOC:BHF, GOC:BHF_miRNA, GOC:TermGenie, GOC:bc, GO_REF:0000058